{
  "gene_symbol": "VAMP8",
  "term_label": "vesicle fusion",
  "term_id": "GO:0006906",
  "gene": "UniProtKB:Q9BV40",
  "gene_name": "Vesicle-associated membrane protein 8"
}